{
  "term_id": "UNKNOWN:0002",
  "gene_name": "Protein FAM228A",
  "term_label": "Unknown biological process",
  "gene": "UniProtKB:Q86W67",
  "gene_symbol": "FAM228A"
}